limonene biosynthetic process [GO:0046250] (biological process) Relationships: is a type of monoterpene biosynthetic process [GO:0043693]; is a type of olefin biosynthetic process [GO:1900674] Definition: The chemical reactions and pathways resulting in the formation of limonene (4-isopropenyl-1-methyl-cyclohexene), a monocyclic monoterpene. Also known as: limonene anabolism, limonene biosynthesis, limonene formation, limonene synthesis Sources: GOC:ai